{
  "gene_symbol": "OR51A7",
  "term_label": "Unknown biological process",
  "gene_name": "Olfactory receptor 51A7",
  "gene": "UniProtKB:Q8NH64",
  "term_id": "UNKNOWN:0002"
}